cellular response to oleic acid [GO:0071400] (biological process) Sources: GOC:mah Definition: Any process that results in a change in state or activity of a cell (in terms of movement, secretion, enzyme production, gene expression, etc.) as a result of an oleic acid stimulus. Also known as: cellular response to oleate Relationships: is a type of response to oleic acid [GO:0034201]; is a type of cellular response to fatty acid [GO:0071398]